{
  "term_label": "cytoskeleton organization",
  "gene_symbol": "FGD3",
  "gene": "UniProtKB:Q5JSP0",
  "gene_name": "FYVE, RhoGEF and PH domain-containing protein 3",
  "term_id": "GO:0007010"
}